regulation of brood size [GO:0060378] (BP) Definition: Any process that modulates brood size. Brood size is the number of progeny that survive embryogenesis and are cared for at one time. Sources: GOC:dph, GOC:tb Relationships: is a type of GO:0044706; is a type of multicellular organismal reproductive process [GO:0048609]; is a type of GO:0065007